regulation of fibroblast proliferation [GO:0048145] (biological process) Subtypes: GO:0048146, negative regulation of fibroblast proliferation [GO:0048147], regulation of hepatic stellate cell proliferation [GO:1904897], regulation of pancreatic stellate cell proliferation [GO:2000229] Definition: Any process that modulates the frequency, rate or extent of multiplication or reproduction of fibroblast cells. Relationships: is a type of regulation of cell population proliferation [GO:0042127]; regulates fibroblast proliferation [GO:0048144] Sources: GOC:jid